{
  "gene": "UniProtKB:O15072",
  "term_label": "metalloendopeptidase activity",
  "gene_symbol": "ADAMTS3",
  "gene_name": "A disintegrin and metalloproteinase with thrombospondin motifs 3",
  "term_id": "GO:0004222"
}